{
  "term_id": "GO:0003729",
  "gene_name": "U6 snRNA-associated Sm-like protein LSm8",
  "gene_symbol": "LSM8",
  "gene": "UniProtKB:O95777",
  "term_label": "mRNA binding"
}